{
  "gene_name": "C-C chemokine receptor type 1",
  "gene_symbol": "CCR1",
  "term_id": "GO:0019722",
  "gene": "UniProtKB:P32246",
  "term_label": "calcium-mediated signaling"
}